response to gamma radiation [GO:0010332] (biological process) Also known as: response to gamma ray, response to gamma-ray photon Sources: GOC:tair_curators Definition: Any process that results in a change in state or activity of a cell or an organism (in terms of movement, secretion, enzyme production, gene expression, etc.) as a result of a gamma radiation stimulus. Gamma radiation is a form of electromagnetic radiation (EMR) or light emission of a specific frequency produced from sub-atomic particle interaction, such as electron-positron annihilation and radioactive decay. Gamma rays are generally characterized as EMR having the highest frequency and energy, and also the shortest wavelength, within the electromagnetic radiation spectrum. Relationships: is a type of response to ionizing radiation [GO:0010212] Subtypes: GO:0071480 Regulation: regulated by regulation of response to gamma radiation [GO:2001228]; negatively regulated by negative regulation of response to gamma radiation [GO:2001229]; positively regulated by positive regulation of response to gamma radiation [GO:2001230]